regulation of protein catabolic process at presynapse, modulating synaptic transmission [GO:0099575] (BP) Note: Note that this term was created for the SynGO project, and will be obsoleted when the SynGO annotations are made in Noctua. Sources: GOC:dos Relationships: is a type of regulation of protein catabolic process [GO:0042176]; is a type of presynaptic modulation of chemical synaptic transmission [GO:0099171] Definition: Any process that modulates synaptic transmission by regulating a catabolic process occurring at a presynapse.